{
  "gene_symbol": "MBD3L4",
  "term_label": "negative regulation of transcription by RNA polymerase II",
  "gene_name": "Putative methyl-CpG-binding domain protein 3-like 4",
  "gene": "UniProtKB:A6NDZ8",
  "term_id": "GO:0000122"
}